2-iminoacetate synthase activity [GO:0036355] (molecular function) References: PMID:17403671 Sources: EC:4.1.99.19, GOC:crds, MetaCyc:RXN-11319 Relationships: is a type of carbon-carbon lyase activity [GO:0016830]; is part of GO:0009228 Definition: Catalysis of the reaction: L-tyrosine + S-adenosyl-L-methionine + reduced acceptor = 2-iminoacetate + 4-methylphenol + 5'-deoxyadenosine + L-methionine + acceptor + 2 H+.